{
  "term_label": "CD8-positive, alpha-beta T cell differentiation involved in immune response",
  "gene": "UniProtKB:O95936",
  "term_id": "GO:0002302",
  "gene_symbol": "EOMES",
  "gene_name": "Eomesodermin homolog"
}